{
  "term_id": "GO:0098839",
  "gene": "UniProtKB:Q9UPU3",
  "gene_symbol": "SORCS3",
  "gene_name": "VPS10 domain-containing receptor SorCS3",
  "term_label": "postsynaptic density membrane"
}